positive regulation of mesodermal cell fate determination [GO:0048336] (BP) Subtypes: GO:0048326, positive regulation of paraxial mesodermal cell fate determination [GO:0048346], positive regulation of lateral mesodermal cell fate determination [GO:0048376], positive regulation of intermediate mesodermal cell fate determination [GO:0048397] Sources: GOC:dgh Relationships: is a type of positive regulation of cell differentiation [GO:0045597]; is a type of regulation of mesodermal cell fate determination [GO:0048334]; is a type of GO:1905935; positively regulates mesodermal cell fate determination [GO:0007500] Also known as: up regulation of mesodermal cell fate determination, up-regulation of mesodermal cell fate determination, upregulation of mesodermal cell fate determination, activation of mesodermal cell fate determination, stimulation of mesodermal cell fate determination Definition: Any process that activates or increases the frequency, rate or extent of mesoderm cell fate determination.